phospholipid-translocating ATPase complex [GO:1990531] (cellular component) Relationships: is a type of transporter complex [GO:1990351] Also known as: APLT complex, P4-ATPase complex, aminophospholipid translocase complex, phospholipid flippase complex, CDC50-DRS2 complex, CRF1-DNF3 complex, DNF3-CRF1 complex, DRS2-CDC50 complex, Dnf1-Lem3 complex, Dnf2-Lem3 complex, Lem3-Dnf1 complex, Lem3p-Dnf1p complex Subtypes: GO:1990530 Definition: A protein complex that functions as a phospholipid-translocating P-Type ATPase. References: PMID:15090616 Sources: GOC:dph, GOC:rb